{
  "term_id": "UNKNOWN:0002",
  "term_label": "Unknown biological process",
  "gene_symbol": "Q8N976",
  "gene_name": "Putative uncharacterized protein FLJ38264",
  "gene": "UniProtKB:Q8N976"
}